{
  "gene": "UniProtKB:Q96B18",
  "term_id": "UNKNOWN:0001",
  "gene_name": "Dapper homolog 3",
  "term_label": "Unknown molecular function",
  "gene_symbol": "DACT3"
}